{
  "term_id": "GO:0007268",
  "gene_name": "Disks large homolog 1",
  "gene_symbol": "DLG1",
  "gene": "UniProtKB:Q12959",
  "term_label": "chemical synaptic transmission"
}